signal recognition particle binding [GO:0005047] (MF) Definition: Binding to a signal recognition particle. Also known as: docking protein, signal recognition particle receptor Sources: ISBN:0198506732 Relationships: is a type of ribonucleoprotein complex binding [GO:0043021] Note: See also the cellular component term 'signal recognition particle, endoplasmic reticulum targeting ; GO:0005786'.